CAAX-protein geranylgeranyltransferase activity [GO:0004662] (molecular function) Relationships: is a type of protein geranylgeranyltransferase activity [GO:0004661] Also known as: GGTase-I activity, GGTaseI activity, geranylgeranyl-diphosphate:protein-cysteine geranyltransferase activity, geranylgeranyltransferase type I activity, protein geranylgeranyltransferase type I, type I protein geranyl-geranyltransferase activity Definition: Catalysis of the reaction: geranylgeranyl diphosphate + protein-cysteine = S-geranylgeranyl-protein + diphosphate. This reaction is the formation of a thioether linkage between the C-1 atom of the geranylgeranyl group and a cysteine residue fourth from the C-terminus of the protein. The protein substrates have the C-terminal sequence CA1A2X, where the terminal residue, X, is preferably leucine and A2 should not be aromatic. Known substrates include most g-subunits of heterotrimeric G proteins and Ras-related GTPases such as members of the Ras and Rac/Rho families. References: PMID:8621375 Sources: EC:2.5.1.59